{
  "term_id": "GO:0003682",
  "gene_symbol": "CHD4",
  "gene": "UniProtKB:Q14839",
  "gene_name": "Chromodomain-helicase-DNA-binding protein 4",
  "term_label": "chromatin binding"
}